{
  "term_id": "UNKNOWN:0003",
  "term_label": "Unknown cellular component",
  "gene_symbol": "ZNF593",
  "gene_name": "Zinc finger protein 593",
  "gene": "UniProtKB:O00488"
}